{
  "gene_symbol": "TRBV5-1",
  "term_id": "GO:0005886",
  "gene_name": "T cell receptor beta variable 5-1",
  "term_label": "plasma membrane",
  "gene": "UniProtKB:A0A578"
}